alpha-1,6-mannosyltransferase activity [GO:0000009] (molecular function) References: PMID:2644248 Sources: GOC:mcc Subtypes: initiation-specific glycolipid 1,6-alpha-mannosyltransferase activity [GO:0033164], GO:0052917, GO:0102704, dol-P-Man:Man(1)GlcN-acyl-PI alpha-1,6-mannosyltransferase activity [GO:0120563] Also known as: 1,6-alpha-mannosyltransferase activity Relationships: is a type of mannosyltransferase activity [GO:0000030] Definition: Catalysis of the transfer of a mannose residue to an oligosaccharide, forming an alpha-(1->6) linkage.